{
  "term_id": "GO:0023051",
  "gene_symbol": "MTURN",
  "gene_name": "Maturin",
  "gene": "UniProtKB:Q8N3F0",
  "term_label": "regulation of signaling"
}